{
  "gene_name": "Inactive ubiquitin carboxyl-terminal hydrolase 53",
  "term_label": "cell-cell junction",
  "gene_symbol": "USP53",
  "gene": "UniProtKB:Q70EK8",
  "term_id": "GO:0005911"
}